alpha-1,3-mannosyltransferase activity [GO:0000033] (molecular function) Definition: Catalysis of the transfer of a mannose residue to an oligosaccharide, forming an alpha-(1->3) linkage. Subtypes: GDP-Man:Man(1)GlcNAc(2)-PP-Dol alpha-1,3-mannosyltransferase activity [GO:0004378], dol-P-Man:Man(5)GlcNAc(2)-PP-Dol alpha-1,3-mannosyltransferase activity [GO:0052925] Relationships: is a type of GO:0000030 References: PMID:10521541 Sources: GOC:mcc